protein serine/threonine phosphatase activity [GO:0004722] (molecular function) Sources: GOC:bf Relationships: is a type of phosphoprotein phosphatase activity [GO:0004721] Regulation: negatively regulated by protein serine/threonine phosphatase inhibitor activity [GO:0004865] Definition: Catalysis of the reaction: protein serine phosphate + H2O = protein serine + phosphate, and protein threonine phosphate + H2O = protein threonine + phosphate. Subtypes: calcium-dependent protein serine/threonine phosphatase activity [GO:0004723], [pyruvate dehydrogenase (acetyl-transferring)]-phosphatase activity [GO:0004741], GO:0008420, myosin phosphatase activity [GO:0017018], MAP kinase serine/threonine phosphatase activity [GO:1990439] Also known as: serine/threonine specific protein phosphatase activity, phosphatase I, phosphatase II, phosphatase III, protein phosphatase type 1 activity, protein phosphatase type 2A activity, protein phosphatase type 2B activity, protein phosphatase type 2C activity, protein phosphatase-1, protein phosphatase-2A, protein phosphatase-2B, protein phosphatase-2C, protein serine phosphatase activity, protein threonine phosphatase activity, magnesium-dependent protein serine/threonine phosphatase activity